{
  "term_label": "glutamatergic synapse",
  "gene_symbol": "SH3GL2",
  "term_id": "GO:0098978",
  "gene": "UniProtKB:Q99962",
  "gene_name": "Endophilin-A1"
}